{
  "term_id": "GO:0017108",
  "gene_symbol": "FAN1",
  "gene": "UniProtKB:Q9Y2M0",
  "gene_name": "Fanconi-associated nuclease 1",
  "term_label": "5'-flap endonuclease activity"
}